{
  "gene": "UniProtKB:P05060",
  "gene_symbol": "CHGB",
  "term_label": "Unknown biological process",
  "term_id": "UNKNOWN:0002",
  "gene_name": "Secretogranin-1"
}